{
  "gene_name": "Collagen alpha-2(VI) chain",
  "gene": "UniProtKB:P12110",
  "term_label": "Unknown biological process",
  "term_id": "UNKNOWN:0002",
  "gene_symbol": "COL6A2"
}